negative regulation of stem cell population maintenance [GO:1902455] (biological process) Definition: Any process that stops, prevents or reduces the frequency, rate or extent of stem cell population maintenance. References: PMID:22969033 Sources: GOC:TermGenie, GOC:hjd Also known as: down regulation of stem cell maintenance, down-regulation of stem cell maintenance, downregulation of stem cell maintenance, inhibition of stem cell maintenance, down regulation of maintenance of pluripotency, down-regulation of maintenance of pluripotency, downregulation of maintenance of pluripotency, inhibition of maintenance of pluripotency, negative regulation of maintenance of pluripotency Relationships: is a type of GO:0051093; is a type of negative regulation of multicellular organismal process [GO:0051241]; is a type of regulation of stem cell population maintenance [GO:2000036]; negatively regulates GO:0019827 Subtypes: GO:1904673